{
  "gene": "UniProtKB:P11926",
  "gene_symbol": "ODC1",
  "term_id": "GO:0033387",
  "term_label": "putrescine biosynthetic process from arginine, via ornithine",
  "gene_name": "Ornithine decarboxylase"
}